regulation of response to osmotic stress [GO:0047484] (biological process) Definition: Any process that modulates the rate or extent of the response to osmotic stress. Relationships: is_a regulation of response to stress [GO:0080134]; regulates response to osmotic stress [GO:0006970] Sources: GOC:ai Subtypes: GO:0106049, GO:1901000